{
  "gene_symbol": "FIGNL1",
  "gene_name": "Fidgetin-like protein 1",
  "term_label": "ATP hydrolysis activity",
  "term_id": "GO:0016887",
  "gene": "UniProtKB:Q6PIW4"
}